N-malonylurea hydrolase activity [GO:0033970] (molecular function) Definition: Catalysis of the reaction: 3-oxo-3-ureidopropanoate + H2O = H+ + malonate + urea. Relationships: is_a hydrolase activity, acting on carbon-nitrogen (but not peptide) bonds, in linear amides [GO:0016811] Also known as: 3-oxo-3-ureidopropanoate amidohydrolase (urea- and malonate-forming) activity, ureidomalonase activity Sources: EC:3.5.1.95, RHEA:17361